alternate splicing of immunoglobulin genes [GO:0002564] (biological process) Definition: The generation of alternate transcripts of immunoglobulin genes through alternate splicing of exons. References: PMID:9185563 Sources: ISBN:0781735149 Relationships: is a type of somatic diversification of immune receptors via alternate splicing [GO:0002563]; is a type of somatic diversification of immunoglobulins [GO:0016445] Also known as: alternate splicing of antibody genes